{
  "term_id": "GO:0009223",
  "gene_symbol": "NT5M",
  "term_label": "pyrimidine deoxyribonucleotide catabolic process",
  "gene_name": "5'(3')-deoxyribonucleotidase, mitochondrial",
  "gene": "UniProtKB:Q9NPB1"
}